cardiac muscle cell proliferation [GO:0060038] (biological process) Definition: The expansion of a cardiac muscle cell population by cell division. Relationships: is_a GO:0014855; is part of cardiac muscle tissue growth [GO:0055017] Also known as: cardiac myocyte proliferation, heart muscle cell proliferation, cardiomyocyte proliferation References: PMID:11161571 Sources: GOC:dph, GOC:rph Regulation: regulated by regulation of cardiac muscle cell proliferation [GO:0060043]; negatively regulated by negative regulation of cardiac muscle cell proliferation [GO:0060044]; positively regulated by positive regulation of cardiac muscle cell proliferation [GO:0060045]